{
  "term_label": "protein localization to Golgi apparatus",
  "gene_symbol": "SYS1",
  "gene": "UniProtKB:Q8N2H4",
  "gene_name": "Protein SYS1 homolog",
  "term_id": "GO:0034067"
}